{
  "gene_symbol": "SMR3B",
  "term_label": "endopeptidase inhibitor activity",
  "term_id": "GO:0004866",
  "gene_name": "Submaxillary gland androgen-regulated protein 3B",
  "gene": "UniProtKB:P02814"
}